pancreatic E cell development [GO:0090105] (biological process) Definition: The process whose specific outcome is the progression of a pancreatic E cell over time, from its formation to the mature structure. Sources: GOC:dph, GOC:tb Relationships: is a type of epithelial cell development [GO:0002064]; is part of pancreatic epsilon cell differentiation [GO:0090104]